{
  "term_id": "GO:0004984",
  "gene_symbol": "OR56A4",
  "gene": "UniProtKB:Q8NGH8",
  "term_label": "olfactory receptor activity",
  "gene_name": "Olfactory receptor 56A4"
}